{
  "gene": "UniProtKB:Q96F45",
  "gene_symbol": "ZNF503",
  "term_id": "UNKNOWN:0001",
  "term_label": "Unknown molecular function",
  "gene_name": "Zinc finger protein 503"
}